{
  "term_id": "UNKNOWN:0001",
  "gene": "UniProtKB:A0A0B4J280",
  "gene_symbol": "TRAV40",
  "term_label": "Unknown molecular function",
  "gene_name": "T cell receptor alpha variable 40"
}